{
  "term_id": "UNKNOWN:0001",
  "gene": "UniProtKB:Q7Z3E5",
  "term_label": "Unknown molecular function",
  "gene_name": "LisH domain-containing protein ARMC9",
  "gene_symbol": "ARMC9"
}